{
  "gene_symbol": "MAPK10",
  "term_label": "cytoplasm",
  "gene_name": "Mitogen-activated protein kinase 10",
  "term_id": "GO:0005737",
  "gene": "UniProtKB:P53779"
}